histidinol-phosphatase activity [GO:0004401] (MF) Definition: Catalysis of the reaction: L-histidinol phosphate + H2O = L-histidinol + phosphate. Also known as: HPpase activity, L-histidinol phosphate phosphatase activity, L-histidinol-phosphate phosphohydrolase activity, histidinol phosphate phosphatase activity, histidinolphosphatase activity, histidinolphosphate phosphatase activity Sources: EC:3.1.3.15, RHEA:14465 Relationships: is a type of phosphatase activity [GO:0016791]